alcohol dehydrogenase (cytochrome c) activity [GO:0052934] (molecular function) Definition: Catalysis of the reaction: 2 [Fe(III)cytochrome c] + a primary alcohol = 2 [Fe(II)cytochrome c] + an aldehyde + 2 H+. Sources: RHEA:51020 Relationships: is a type of oxidoreductase activity, acting on the CH-OH group of donors, cytochrome as acceptor [GO:0016898] Also known as: alcohol dehydrogenase (acceptor) activity, PQQ-dependent alcohol dehydrogenase activity, alcohol:cytochrome c oxidoreductase activity, 2-chloroethanol:cytochrome c oxidoreductase activity, ethanol:cytochrome c oxidoreductase activity, alcohol:(acceptor) oxidoreductase activity, alcohol:acceptor oxidoreductase activity, quinoprotein alcohol dehydrogenase activity